{
  "gene": "UniProtKB:Q9BX70",
  "gene_symbol": "BTBD2",
  "term_label": "neurogenesis",
  "gene_name": "BTB_POZ domain-containing protein 2",
  "term_id": "GO:0022008"
}